positive regulation of nitrogen utilization [GO:0045848] (biological process) Relationships: is a type of regulation of nitrogen utilization [GO:0006808]; is a type of positive regulation of response to nutrient levels [GO:0032109]; positively regulates GO:0019740 Sources: GOC:go_curators Definition: Any process that activates or increases the frequency, rate or extent of nitrogen utilization. Subtypes: positive regulation of ammonia assimilation cycle [GO:2001250] Also known as: up regulation of nitrogen utilization, up-regulation of nitrogen utilization, upregulation of nitrogen utilization, activation of nitrogen utilization, stimulation of nitrogen utilization